stringent response [GO:0015968] (biological process) Definition: A specific global change in the metabolism of a bacterial cell (the downregulation of nucleic acid and protein synthesis, and the simultaneous upregulation of protein degradation and amino acid synthesis) as a result of starvation. Relationships: is a type of cellular response to starvation [GO:0009267] References: PMID:11282471 Sources: GOC:jl, ISBN:0124325653